positive regulation of antigen processing and presentation of peptide antigen via MHC class II [GO:0002588] (biological process) Definition: Any process that activates or increases the frequency, rate, or extent of antigen processing and presentation of peptide antigen via MHC class II. Relationships: is a type of positive regulation of antigen processing and presentation of peptide or polysaccharide antigen via MHC class II [GO:0002582]; is a type of GO:0002585; is a type of regulation of antigen processing and presentation of peptide antigen via MHC class II [GO:0002586]; positively regulates antigen processing and presentation of peptide antigen via MHC class II [GO:0002495] Sources: GOC:add Also known as: positive regulation of peptide antigen processing and presentation via MHC class II, up regulation of antigen processing and presentation of peptide antigen via MHC class II, up-regulation of antigen processing and presentation of peptide antigen via MHC class II, upregulation of antigen processing and presentation of peptide antigen via MHC class II, activation of antigen processing and presentation of peptide antigen via MHC class II, stimulation of antigen processing and presentation of peptide antigen via MHC class II